regulation of synaptic vesicle membrane organization [GO:1901632] (biological process) References: PMID:22426000 Sources: GOC:TermGenie Also known as: regulation of synaptic vesicle membrane organisation, regulation of SLMV biogenesis, regulation of synaptic vesicle membrane organization and biogenesis Definition: Any process that modulates the frequency, rate or extent of synaptic vesicle membrane organization. Subtypes: GO:0031630, negative regulation of synaptic vesicle membrane organization [GO:1901633], positive regulation of synaptic vesicle membrane organization [GO:1901634] Relationships: is a type of GO:0051128; regulates GO:0048499